UTP biosynthetic process [GO:0006228] (biological process) Also known as: UTP anabolism, UTP biosynthesis, UTP formation, UTP synthesis Definition: The chemical reactions and pathways resulting in the formation of UTP, uridine (5'-)triphosphate. Sources: ISBN:0198506732 Relationships: is a type of GO:0009209; is a type of GO:0009220; is a type of GO:0046051